{
  "term_label": "plasma membrane",
  "gene": "UniProtKB:P43353",
  "gene_name": "Aldehyde dehydrogenase family 3 member B1",
  "gene_symbol": "ALDH3B1",
  "term_id": "GO:0005886"
}